{
  "term_id": "UNKNOWN:0002",
  "term_label": "Unknown biological process",
  "gene_symbol": "FAM86B2",
  "gene_name": "Putative protein N-methyltransferase FAM86B2",
  "gene": "UniProtKB:P0C5J1"
}